{
  "gene": "UniProtKB:O60237",
  "gene_name": "Protein phosphatase 1 regulatory subunit 12B",
  "gene_symbol": "PPP1R12B",
  "term_label": "cytoplasm",
  "term_id": "GO:0005737"
}